{
  "term_label": "nucleus",
  "term_id": "GO:0005634",
  "gene_name": "Interferon-stimulated gene 20 kDa protein",
  "gene_symbol": "ISG20",
  "gene": "UniProtKB:Q96AZ6"
}